{
  "gene": "UniProtKB:Q5JVL4",
  "gene_name": "EF-hand domain-containing protein 1",
  "term_id": "GO:0000281",
  "gene_symbol": "EFHC1",
  "term_label": "mitotic cytokinesis"
}